{
  "gene_name": "Galectin-10",
  "gene": "UniProtKB:Q05315",
  "term_id": "GO:0030246",
  "term_label": "carbohydrate binding",
  "gene_symbol": "CLC"
}